{
  "gene": "UniProtKB:P13631",
  "gene_symbol": "RARG",
  "term_label": "cell differentiation",
  "term_id": "GO:0030154",
  "gene_name": "Retinoic acid receptor gamma"
}